{
  "gene_name": "Coiled-coil domain-containing protein 13",
  "term_id": "GO:0034451",
  "gene_symbol": "CCDC13",
  "term_label": "centriolar satellite",
  "gene": "UniProtKB:Q8IYE1"
}